{
  "gene_name": "Protein FAM124B",
  "term_id": "GO:0005654",
  "term_label": "nucleoplasm",
  "gene": "UniProtKB:Q9H5Z6",
  "gene_symbol": "FAM124B"
}